{
  "gene_name": "T cell receptor alpha variable 22",
  "term_id": "UNKNOWN:0003",
  "term_label": "Unknown cellular component",
  "gene_symbol": "TRAV22",
  "gene": "UniProtKB:A0A0B4J277"
}